{
  "gene_name": "Doublecortin domain-containing protein 2",
  "term_label": "regulation of cilium assembly",
  "term_id": "GO:1902017",
  "gene_symbol": "DCDC2",
  "gene": "UniProtKB:Q9UHG0"
}